{
  "term_id": "GO:0006412",
  "gene": "UniProtKB:Q4U2R6",
  "gene_symbol": "MRPL51",
  "gene_name": "Large ribosomal subunit protein mL51",
  "term_label": "translation"
}